{
  "gene_symbol": "ADPRS",
  "term_label": "mitochondrion",
  "gene": "UniProtKB:Q9NX46",
  "term_id": "GO:0005739",
  "gene_name": "ADP-ribosylhydrolase ARH3"
}